{
  "gene": "UniProtKB:Q9BVG9",
  "term_label": "Unknown molecular function",
  "gene_name": "Phosphatidylserine synthase 2",
  "gene_symbol": "PTDSS2",
  "term_id": "UNKNOWN:0001"
}